{
  "term_id": "GO:0098609",
  "term_label": "cell-cell adhesion",
  "gene_symbol": "IGDCC3",
  "gene_name": "Immunoglobulin superfamily DCC subclass member 3",
  "gene": "UniProtKB:Q8IVU1"
}